{
  "gene_name": "Stabilizer of axonemal microtubules 1",
  "gene": "UniProtKB:Q8IYX7",
  "term_label": "axonemal microtubule",
  "term_id": "GO:0005879",
  "gene_symbol": "SAXO1"
}